{
  "term_id": "GO:0098978",
  "gene_symbol": "SLITRK4",
  "gene_name": "SLIT and NTRK-like protein 4",
  "gene": "UniProtKB:Q8IW52",
  "term_label": "glutamatergic synapse"
}